{
  "gene_name": "PHD finger protein 19",
  "term_label": "chromatin binding",
  "gene": "UniProtKB:Q5T6S3",
  "gene_symbol": "PHF19",
  "term_id": "GO:0003682"
}